{
  "gene_symbol": "POTEE",
  "term_id": "GO:0007409",
  "term_label": "axonogenesis",
  "gene": "UniProtKB:Q6S8J3",
  "gene_name": "POTE ankyrin domain family member E"
}